{
  "gene_name": "PRA1 family protein 2",
  "term_label": "Unknown molecular function",
  "term_id": "UNKNOWN:0001",
  "gene": "UniProtKB:O60831",
  "gene_symbol": "PRAF2"
}